positive regulation of amino acid uptake involved in synaptic transmission [GO:0051943] (biological process) Relationships: is a type of GO:0051582; is a type of GO:0051941; is a type of GO:0051957; positively regulates GO:0051933 Also known as: positive regulation of amino acid neurotransmitter reuptake, positive regulation of amino acid neurotransmitter uptake, stimulation of amino acid uptake during transmission of nerve impulse, activation of amino acid uptake during transmission of nerve impulse, up regulation of amino acid uptake during transmission of nerve impulse, up-regulation of amino acid uptake during transmission of nerve impulse, upregulation of amino acid uptake during transmission of nerve impulse Definition: Any process that activates, maintains or increases the frequency, rate or extent of the directed movement of amino acid neurotransmitters into a neuron or glial cell. Subtypes: positive regulation of gamma-aminobutyric acid uptake involved in transmission of nerve impulse [GO:0051950], positive regulation of glutamate uptake involved in transmission of nerve impulse [GO:0051951] Sources: GOC:ai